activation of recombination (HML) [GO:0007536] (biological process) References: PMID:9928492 Sources: GOC:mah Relationships: is_a donor selection [GO:0007535]; is a type of positive regulation of DNA recombination [GO:0045911] Definition: The activation of recombination at a mating type locus, such that it is used in preference to the other donor locus for mating type switching; exemplified by the HML locus and surrounding sequences on Chromosome III in Saccharomyces cerevisiae.